{
  "gene": "UniProtKB:Q9Y5B6",
  "gene_name": "PAX3- and PAX7-binding protein 1",
  "gene_symbol": "PAXBP1",
  "term_label": "Unknown molecular function",
  "term_id": "UNKNOWN:0001"
}